{
  "gene_symbol": "SOS1",
  "gene": "UniProtKB:Q07889",
  "term_id": "GO:0005085",
  "gene_name": "Son of sevenless homolog 1",
  "term_label": "guanyl-nucleotide exchange factor activity"
}